{
  "term_label": "Unknown molecular function",
  "gene_name": "Gastrokine-1",
  "gene_symbol": "GKN1",
  "gene": "UniProtKB:Q9NS71",
  "term_id": "UNKNOWN:0001"
}